{
  "gene_name": "Band 3 anion transport protein",
  "gene": "UniProtKB:P02730",
  "term_id": "GO:0016323",
  "gene_symbol": "SLC4A1",
  "term_label": "basolateral plasma membrane"
}